{
  "gene": "UniProtKB:Q9UKT4",
  "gene_symbol": "FBXO5",
  "term_id": "GO:0007088",
  "gene_name": "F-box only protein 5",
  "term_label": "regulation of mitotic nuclear division"
}